{
  "gene_symbol": "LSM3",
  "gene_name": "U6 snRNA-associated Sm-like protein LSm3",
  "gene": "UniProtKB:P62310",
  "term_label": "U6 snRNP",
  "term_id": "GO:0005688"
}